{
  "term_label": "Unknown molecular function",
  "gene_name": "Platelet glycoprotein Ib beta chain",
  "term_id": "UNKNOWN:0001",
  "gene": "UniProtKB:P13224",
  "gene_symbol": "GP1BB"
}